regulation of Atg1/ULK1 kinase complex assembly [GO:1905864] (biological process) Subtypes: negative regulation of Atg1/ULK1 kinase complex assembly [GO:1905865], positive regulation of Atg1/ULK1 kinase complex assembly [GO:1905866] Also known as: regulation of ATG1 kinase complex assembly, regulation of ATG1 kinase complex formation, regulation of ATG1-ATG13 complex assembly, regulation of ATG1-ATG13 complex formation, regulation of ATG1/ULK1 kinase complex formation, regulation of ATG1/ULK1 signaling complex assembly, regulation of ATG1/ULK1 signaling complex formation, regulation of Atg1p signalling complex assembly, regulation of Atg1p signalling complex formation, regulation of ULK1 signaling complex assembly, regulation of ULK1 signaling complex formation, regulation of ULK1-ATG13-FIP200 complex assembly, regulation of ULK1-ATG13-FIP200 complex formation, regulation of ULK1-ATG13-RB1CC1 complex assembly, regulation of ULK1-ATG13-RB1CC1 complex formation References: PMID:26567215 Sources: GOC:TermGenie, GOC:autophagy, GOC:mf, GO_REF:0000058 Definition: Any process that modulates the frequency, rate or extent of Atg1/ULK1 kinase complex assembly. Relationships: is a type of regulation of protein-containing complex assembly [GO:0043254]; regulates Atg1/ULK1 kinase complex assembly [GO:1904745]